G protein-coupled receptor signaling pathway involved in dauer larval development [GO:1904066] (biological process) Relationships: is a type of G protein-coupled receptor signaling pathway [GO:0007186]; BFO_0000050 dauer larval development [GO:0040024] References: PMID:22665789 Sources: GOC:TermGenie, GOC:kmv, GO_REF:0000060 Also known as: G protein coupled receptor protein signaling pathway involved in dauer larval development, G protein coupled receptor protein signalling pathway involved in dauer larval development, G-protein coupled receptor protein signal transduction involved in dauer larval development, G-protein coupled receptor protein signaling pathway involved in dauer larval development, G-protein coupled receptor signalling pathway involved in dauer larval development, G-protein-coupled receptor protein signalling pathway involved in dauer larval development, GPCR signaling pathway involved in dauer larval development, GPCR signalling pathway involved in dauer larval development Definition: Any G protein-coupled receptor signaling pathway that is involved in dauer larval development.